{
  "gene_symbol": "SOX17",
  "term_id": "GO:0005634",
  "gene_name": "Transcription factor SOX-17",
  "term_label": "nucleus",
  "gene": "UniProtKB:Q9H6I2"
}